{
  "gene_name": "Cyclin-dependent kinase 9",
  "gene": "UniProtKB:P50750",
  "term_label": "cyclin-dependent protein kinase holoenzyme complex",
  "term_id": "GO:0000307",
  "gene_symbol": "CDK9"
}